{
  "term_label": "replication fork arrest",
  "term_id": "GO:0043111",
  "gene_symbol": "TIMELESS",
  "gene": "UniProtKB:Q9UNS1",
  "gene_name": "Protein timeless homolog"
}